arylamine N-acetyltransferase activity [GO:0004060] (molecular function) Relationships: is a type of N-acetyltransferase activity [GO:0008080] Definition: Catalysis of the reaction: acetyl-CoA + an arylamine = CoA + an N-acetylarylamine. Also known as: 2-naphthylamine N-acetyltransferase activity, 4-aminobiphenyl N-acetyltransferase activity, acetyl CoA-arylamine N-acetyltransferase activity, acetyl-CoA:arylamine N-acetyltransferase activity, arylamine acetylase activity, arylamine acetyltransferase activity, beta-naphthylamine N-acetyltransferase activity, indoleamine N-acetyltransferase activity, p-aminosalicylate N-acetyltransferase activity Sources: EC:2.3.1.5